{
  "gene_symbol": "GPM6A",
  "term_label": "axonal growth cone",
  "gene": "UniProtKB:P51674",
  "gene_name": "Neuronal membrane glycoprotein M6-a",
  "term_id": "GO:0044295"
}